{
  "gene_symbol": "NRIP3",
  "term_label": "cytoplasm",
  "gene_name": "Nuclear receptor-interacting protein 3",
  "term_id": "GO:0005737",
  "gene": "UniProtKB:Q9NQ35"
}